pyripyropene A biosynthetic process [GO:0140652] (biological process) Relationships: is a type of GO:0016106 Definition: The chemical reactions and pathways resulting in the formation of pyripyropene A. Also known as: pyripyropene A anabolism, pyripyropene A biosynthesis, pyripyropene A formation, pyripyropene A synthesis References: PMID:21224862, PMID:26019565 Sources: GOC:ach